{
  "gene_symbol": "LDHAL6B",
  "gene_name": "L-lactate dehydrogenase A-like 6B",
  "term_id": "GO:0042867",
  "term_label": "pyruvate catabolic process",
  "gene": "UniProtKB:Q9BYZ2"
}